{
  "term_id": "GO:0070588",
  "term_label": "calcium ion transmembrane transport",
  "gene": "UniProtKB:Q71RS6",
  "gene_name": "Sodium_potassium_calcium exchanger 5",
  "gene_symbol": "SLC24A5"
}